{
  "term_id": "GO:0008076",
  "gene_symbol": "KCNB2",
  "gene_name": "Potassium voltage-gated channel subfamily B member 2",
  "gene": "UniProtKB:Q92953",
  "term_label": "voltage-gated potassium channel complex"
}